thymidine biosynthetic process [GO:0046105] (biological process) Definition: The chemical reactions and pathways resulting in the formation of thymidine, deoxyribosylthymine thymine 2-deoxyriboside, a deoxynucleoside very widely distributed but occurring almost entirely as phosphoric esters in deoxynucleotides and deoxyribonucleic acid, DNA. Sources: GOC:go_curators Also known as: deoxyribosylthymine biosynthesis, deoxyribosylthymine biosynthetic process, thymidine anabolism, thymidine biosynthesis, thymidine formation, thymidine synthesis Relationships: is a type of GO:0046104; is a type of pyrimidine deoxyribonucleoside biosynthetic process [GO:0046126]